{
  "gene_symbol": "OSBPL7",
  "gene": "UniProtKB:Q9BZF2",
  "term_label": "plasma membrane",
  "gene_name": "Oxysterol-binding protein-related protein 7",
  "term_id": "GO:0005886"
}